{
  "gene": "UniProtKB:Q9UHW9",
  "term_id": "GO:0055075",
  "gene_symbol": "SLC12A6",
  "term_label": "potassium ion homeostasis",
  "gene_name": "Solute carrier family 12 member 6"
}